{
  "term_id": "UNKNOWN:0003",
  "gene_symbol": "WDR47",
  "term_label": "Unknown cellular component",
  "gene": "UniProtKB:O94967",
  "gene_name": "WD repeat-containing protein 47"
}